regulation of termination of RNA polymerase I transcription [GO:2000730] (biological process) Sources: GOC:obol Also known as: regulation of RNA polymerase I transcription termination, regulation of transcription termination from Pol I promoter, regulation of transcription termination from RNA polymerase I promoter Definition: Any process that modulates the frequency, rate or extent of termination of RNA polymerase I transcription. Relationships: is a type of regulation of transcription by RNA polymerase I [GO:0006356]; is a type of regulation of termination of DNA-templated transcription [GO:0031554]; regulates GO:0006363 Subtypes: negative regulation of termination of RNA polymerase I transcription [GO:2000731], positive regulation of termination of RNA polymerase I transcription [GO:2000732]